pericardium development [GO:0060039] (biological process) References: PMID:15138308, PMID:16376438 Sources: GOC:dph, GOC:rph Definition: The process whose specific outcome is the progression of the pericardium over time, from its formation to the mature structure. The pericardium is a double-walled sac that contains the heart and the roots of the aorta, vena cava and the pulmonary artery. Relationships: is a type of epithelium development [GO:0060429]; BFO_0000050 heart development [GO:0007507]